{
  "gene": "UniProtKB:Q9H7X2",
  "term_label": "Unknown biological process",
  "term_id": "UNKNOWN:0002",
  "gene_symbol": "C1orf115",
  "gene_name": "Required for drug-induced death protein 1"
}